{
  "gene_symbol": "SCHIP1",
  "term_label": "Unknown molecular function",
  "gene_name": "Schwannomin-interacting protein 1",
  "gene": "UniProtKB:P0DPB3",
  "term_id": "UNKNOWN:0001"
}